{
  "gene": "UniProtKB:P12955",
  "gene_symbol": "PEPD",
  "gene_name": "Xaa-Pro dipeptidase",
  "term_label": "proteolysis",
  "term_id": "GO:0006508"
}